transmembrane transport [GO:0055085] (biological process) Note: Transmembrane transport is the transport of a solute across a lipid bilayer. Note that transport through the nuclear pore complex is not transmembrane because the nuclear membrane is a double membrane and is not traversed. For transport through the nuclear pore, consider instead the term 'nucleocytoplasmic transport ; GO:0006913' and its children. Note also that this term is not intended for use in annotating lateral movement within membranes. Also known as: membrane transport, ATP hydrolysis coupled transmembrane transport Sources: GOC:dph, GOC:jid Definition: The process in which a solute is transported across a lipid bilayer, from one side of a membrane to the other. Regulation: regulated by regulation of transmembrane transport [GO:0034762]; negatively regulated by GO:0034763; positively regulated by positive regulation of transmembrane transport [GO:0034764] Relationships: is a type of transport [GO:0006810]; is a type of cellular process [GO:0009987] Subtypes: sulfite transmembrane transport [GO:0000316], GO:0001407, amino acid transmembrane transport [GO:0003333], xenobiotic transmembrane transport [GO:0006855], antimonite transmembrane transport [GO:0015699], nitrate transmembrane transport [GO:0015706], tartrate transmembrane transport [GO:0015745], nucleotide-sugar transmembrane transport [GO:0015780], polyol transmembrane transport [GO:0015791], GO:0015794, tetracycline transmembrane transport [GO:0015904], bicyclomycin transmembrane transport [GO:0015905], carbohydrate transmembrane transport [GO:0034219], GO:0034220, vacuolar transmembrane transport [GO:0034486], carbon dioxide transmembrane transport [GO:0035378], sterol transmembrane transport [GO:0035382], phosphate ion transmembrane transport [GO:0035435], triose phosphate transmembrane transport [GO:0035436], GO:0035445, vitamin transmembrane transport [GO:0035461], oligopeptide transmembrane transport [GO:0035672], RNA import into mitochondrion [GO:0035927], alkanesulfonate transmembrane transport [GO:0042918], GO:0045117, xenobiotic export from cell [GO:0046618], cytosol to endoplasmic reticulum transport [GO:0046967], glycerol-2-phosphate transmembrane transport [GO:0070811], GO:0071806, GO:0071918, phytochelatin transmembrane transport [GO:0071994], ammonium transmembrane transport [GO:0072488], methylammonium transmembrane transport [GO:0072489], GO:0072530, GO:0072531, endoplasmic reticulum to cytosol auxin transport [GO:0080162], hydrogen peroxide transmembrane transport [GO:0080170], plasma membrane selenite transport [GO:0097080], import across plasma membrane [GO:0098739], export across plasma membrane [GO:0140115], export across cell outer membrane [GO:0140317], cytosol to Golgi apparatus transport [GO:0140820], lipoate transmembrane transport [GO:0170006], nucleoside transmembrane transport [GO:1901642], nucleotide transmembrane transport [GO:1901679], GO:1901684, GO:1901962, polyamine transmembrane transport [GO:1902047], sulfate transmembrane transport [GO:1902358], (+)-abscisic acid D-glucopyranosyl ester transmembrane transport [GO:1902418], aluminum ion transmembrane transport [GO:1902602], carnitine transmembrane transport [GO:1902603], O-acyl-L-carnitine transmembrane transport [GO:1902616], carboxylic acid transmembrane transport [GO:1905039], mitochondrial transmembrane transport [GO:1990542]